{
  "term_id": "GO:0042802",
  "term_label": "identical protein binding",
  "gene": "UniProtKB:P46926",
  "gene_symbol": "GNPDA1",
  "gene_name": "Glucosamine-6-phosphate isomerase 1"
}